{
  "term_label": "Unknown molecular function",
  "gene_symbol": "QTRT2",
  "gene": "UniProtKB:Q9H974",
  "term_id": "UNKNOWN:0001",
  "gene_name": "Queuine tRNA-ribosyltransferase accessory subunit 2"
}